{
  "gene": "UniProtKB:Q9BYQ4",
  "gene_symbol": "KRTAP9-2",
  "term_id": "UNKNOWN:0003",
  "gene_name": "Keratin-associated protein 9-2",
  "term_label": "Unknown cellular component"
}